{
  "gene_name": "Meiosis-specific protein MEI4",
  "term_label": "oogenesis",
  "gene_symbol": "MEI4",
  "gene": "UniProtKB:A8MW99",
  "term_id": "GO:0048477"
}